{
  "gene_name": "Gamma-aminobutyric acid receptor-associated protein-like 1",
  "gene": "UniProtKB:Q9H0R8",
  "term_label": "autophagosome maturation",
  "gene_symbol": "GABARAPL1",
  "term_id": "GO:0097352"
}